regulation of neuronal action potential [GO:0098908] (biological process) Subtypes: negative regulation of neuronal action potential [GO:1904456], positive regulation of neuronal action potential [GO:1904457] Also known as: generation of action potential Sources: GOC:dph, GOC:isa_complete, GOC:tb Relationships: is a type of regulation of transmission of nerve impulse [GO:0051969]; is a type of regulation of action potential [GO:0098900]; RO_0002211 neuronal action potential [GO:0019228] Definition: Any process that modulates the frequency, rate or extent of action potential creation, propagation or termination in a neuron. This typically occurs via modulation of the activity or expression of voltage-gated ion channels.